long-term synaptic depression [GO:0060292] (biological process) Regulation: regulated by GO:1900452; negatively regulated by negative regulation of long-term synaptic depression [GO:1900453]; positively regulated by positive regulation of long-term synaptic depression [GO:1900454] Definition: A process that modulates synaptic plasticity such that synapses are changed resulting in the decrease in the rate, or frequency of synaptic transmission at the synapse. Sources: GOC:dgh, GOC:dph Also known as: long term depression, long term synaptic depression, LTD Relationships: is a type of regulation of synaptic plasticity [GO:0048167]; is a type of GO:0050805